{
  "gene": "UniProtKB:P49910",
  "gene_symbol": "ZNF165",
  "gene_name": "Zinc finger protein 165",
  "term_label": "RNA polymerase II cis-regulatory region sequence-specific DNA binding",
  "term_id": "GO:0000978"
}